{
  "gene": "UniProtKB:P20592",
  "gene_symbol": "MX2",
  "term_label": "plasma membrane",
  "gene_name": "Interferon-induced GTP-binding protein Mx2",
  "term_id": "GO:0005886"
}